positive regulation of cardiac muscle myoblast proliferation [GO:0110024] (biological process) References: PMID:26512644 Sources: GOC:BHF, GOC:BHF_miRNA, GOC:rph Definition: Any process that activates or increases the frequency, rate or extent of cardiac muscle myoblast proliferation. Relationships: is a type of regulation of cardiac muscle myoblast proliferation [GO:0110022]; is a type of GO:2000288; positively regulates cardiac muscle myoblast proliferation [GO:0110021]